{
  "gene": "UniProtKB:Q96B33",
  "term_label": "plasma membrane",
  "gene_name": "Claudin-23",
  "term_id": "GO:0005886",
  "gene_symbol": "CLDN23"
}